alkane biosynthetic process [GO:0043447] (biological process) Regulation: regulated by regulation of alkane biosynthetic process [GO:1901577]; negatively regulated by negative regulation of alkane biosynthetic process [GO:1901578]; positively regulated by positive regulation of alkane biosynthetic process [GO:1901579] Also known as: alkane anabolism, alkane biosynthesis, alkane formation, alkane synthesis Sources: GOC:jl, Wikipedia:Alkane Subtypes: methanogenesis [GO:0015948], tridecane biosynthetic process [GO:1900632], pentadecane biosynthetic process [GO:1900634], heptadecane biosynthetic process [GO:1900636] Relationships: is a type of hydrocarbon biosynthetic process [GO:0120251] Definition: The chemical reactions and pathways resulting in the formation of an alkane, any acyclic branched or unbranched hydrocarbon having the general formula CnH2n+2.